{
  "gene": "UniProtKB:P41743",
  "term_label": "intracellular signal transduction",
  "gene_symbol": "PRKCI",
  "term_id": "GO:0035556",
  "gene_name": "Protein kinase C iota type"
}